old cell tip after activation of bipolar cell growth [GO:0035842] (cellular component) Sources: GOC:expert_jd, GOC:mah Definition: A cell tip which has existed for at least one complete cell cycle, and at which polarized growth occurs, which is part of a cell that has activated bipolar cell growth (i.e. in which new end take-off, NETO, has taken place). For example, in fission yeast the cell end that existed prior to cell division grows immediately after division, and contains a distinctive complement of proteins including actin cytoskeletal structures. Also known as: post-NETO old cell end, post-NETO old cell tip, post-new end take-off old cell tip Relationships: is a type of old growing cell tip [GO:0035840]